{
  "gene_symbol": "KASH5",
  "gene_name": "Protein KASH5",
  "term_id": "GO:0051653",
  "gene": "UniProtKB:Q8N6L0",
  "term_label": "spindle localization"
}